{
  "gene_symbol": "POTEF",
  "term_label": "synapse",
  "gene_name": "POTE ankyrin domain family member F",
  "gene": "UniProtKB:A5A3E0",
  "term_id": "GO:0045202"
}